catechol 2,3-dioxygenase activity [GO:0018577] (molecular function) Relationships: is a type of oxidoreductase activity, acting on single donors with incorporation of molecular oxygen, incorporation of two atoms of oxygen [GO:0016702] Sources: RHEA:17337 Definition: Catalysis of the reaction: catechol + O2 = 2-hydroxymuconate semialdehyde. Also known as: 2,3-pyrocatechase activity, catechol 2,3-oxygenase, catechol oxygenase, catechol:oxygen 2,3-oxidoreductase (decyclizing), cato2ase activity, metapyrocatechase activity, pyrocatechol 2,3-dioxygenase